fucosidase activity [GO:0015928] (MF) Relationships: is a type of hydrolase activity, hydrolyzing O-glycosyl compounds [GO:0004553] Sources: GOC:ai Definition: Catalysis of the hydrolysis of fucosyl compounds, substances containing a group derived from a cyclic form of fucose or a fucose derivative. Subtypes: alpha-L-fucosidase activity [GO:0004560], GO:0033907